{
  "gene_symbol": "QPCT",
  "gene_name": "Glutaminyl-peptide cyclotransferase",
  "gene": "UniProtKB:Q16769",
  "term_id": "UNKNOWN:0002",
  "term_label": "Unknown biological process"
}